{
  "gene": "UniProtKB:O15258",
  "term_id": "GO:0006621",
  "term_label": "protein retention in ER lumen",
  "gene_symbol": "RER1",
  "gene_name": "Protein RER1"
}